{
  "term_id": "GO:0016251",
  "term_label": "RNA polymerase II general transcription initiation factor activity",
  "gene_symbol": "GTF2E2",
  "gene_name": "Transcription initiation factor IIE subunit beta",
  "gene": "UniProtKB:P29084"
}